{
  "gene_symbol": "PBLD",
  "term_id": "UNKNOWN:0002",
  "term_label": "Unknown biological process",
  "gene": "UniProtKB:P30039",
  "gene_name": "Phenazine biosynthesis-like domain-containing protein"
}